{
  "gene": "UniProtKB:Q9BQ65",
  "gene_symbol": "USB1",
  "gene_name": "U6 snRNA phosphodiesterase 1",
  "term_id": "GO:0005634",
  "term_label": "nucleus"
}